negative regulation of antibacterial peptide secretion [GO:0002798] (BP) Sources: GOC:add Definition: Any process that stops, prevents, or reduces the frequency, rate, or extent of antibacterial peptide secretion. Relationships: is a type of negative regulation of antibacterial peptide production [GO:0002787]; is a type of negative regulation of antimicrobial peptide secretion [GO:0002795]; is a type of regulation of antibacterial peptide secretion [GO:0002797]; negatively regulates antibacterial peptide secretion [GO:0002779] Also known as: down regulation of antibacterial peptide secretion, down-regulation of antibacterial peptide secretion, downregulation of antibacterial peptide secretion, inhibition of antibacterial peptide secretion